negative regulation of DNA amplification [GO:1904524] (BP) Relationships: is a type of regulation of DNA amplification [GO:1904523]; is a type of negative regulation of DNA biosynthetic process [GO:2000279]; negatively regulates DNA amplification [GO:0006277] Also known as: down regulation of DNA amplification, down-regulation of DNA amplification, downregulation of DNA amplification, inhibition of DNA amplification References: PMID:26195783 Sources: GOC:TermGenie, GO_REF:0000058 Definition: Any process that stops, prevents or reduces the frequency, rate or extent of DNA amplification.